{
  "gene_symbol": "TSFM",
  "term_id": "GO:0070125",
  "gene": "UniProtKB:P43897",
  "gene_name": "Elongation factor Ts, mitochondrial",
  "term_label": "mitochondrial translational elongation"
}